{
  "term_id": "UNKNOWN:0003",
  "gene": "UniProtKB:Q8IZ16",
  "term_label": "Unknown cellular component",
  "gene_name": "Sperm acrosome developmental regulator",
  "gene_symbol": "SPACDR"
}